acetyl-CoA transport [GO:0015876] (biological process) Subtypes: GO:0035348 Relationships: is a type of GO:0015916 Definition: The directed movement of acetyl-CoA into, out of or within a cell, or between cells, by means of some agent such as a transporter or pore. Acetyl-CoA is a derivative of coenzyme A in which the sulfhydryl group is acetylated; it is a metabolite derived from several pathways (e.g. glycolysis, fatty acid oxidation, amino-acid catabolism) and is further metabolized by the tricarboxylic acid cycle. It is a key intermediate in lipid and terpenoid biosynthesis. Sources: GOC:ai